organellar ribosome [GO:0000313] (cellular component) Sources: GOC:mah, GOC:mcc Relationships: is a type of ribosome [GO:0005840]; BFO_0000050 organelle [GO:0043226] Definition: A ribosome contained within a subcellular membrane-bounded organelle. Subtypes: mitochondrial ribosome [GO:0005761], plastid ribosome [GO:0009547]